{
  "gene_symbol": "HMGCLL1",
  "term_id": "GO:0004419",
  "gene": "UniProtKB:Q8TB92",
  "term_label": "hydroxymethylglutaryl-CoA lyase activity",
  "gene_name": "3-hydroxy-3-methylglutaryl-CoA lyase, cytoplasmic"
}